{
  "term_id": "GO:0005965",
  "gene": "UniProtKB:P49356",
  "gene_symbol": "FNTB",
  "term_label": "protein farnesyltransferase complex",
  "gene_name": "Protein farnesyltransferase subunit beta"
}